{
  "term_id": "UNKNOWN:0003",
  "gene_name": "Solute carrier family 25 member 34",
  "term_label": "Unknown cellular component",
  "gene": "UniProtKB:Q6PIV7",
  "gene_symbol": "SLC25A34"
}